{
  "term_id": "UNKNOWN:0002",
  "gene_name": "Single-strand selective monofunctional uracil DNA glycosylase",
  "gene_symbol": "SMUG1",
  "term_label": "Unknown biological process",
  "gene": "UniProtKB:Q53HV7"
}